stearoyl-[ACP] desaturase activity [GO:0045300] (molecular function) Also known as: acyl-[acyl-carrier-protein] desaturase activity, acyl-acyl-carrier-protein desaturase activity, acyl-acyl-carrier-protein, hydrogen-donor:oxygen oxidoreductase activity, stearyl acyl carrier protein desaturase activity, stearyl-ACP desaturase activity Relationships: is_a oxidoreductase activity, acting on paired donors, with oxidation of a pair of donors resulting in the reduction of molecular oxygen to two molecules of water [GO:0016717] Definition: Catalysis of the reaction: 2 H+ + O2 + octadecanoyl-[ACP] + 2 reduced [2Fe-2S]-[ferredoxin] = (9Z)-octadecenoyl-[ACP] + 2 H2O + 2 oxidized [2Fe-2S]-[ferredoxin]. Sources: RHEA:11776